{
  "term_id": "GO:0000981",
  "gene_name": "Zinc finger protein 419",
  "term_label": "DNA-binding transcription factor activity, RNA polymerase II-specific",
  "gene": "UniProtKB:Q96HQ0",
  "gene_symbol": "ZNF419"
}